{
  "gene": "UniProtKB:O75489",
  "gene_symbol": "NDUFS3",
  "term_id": "UNKNOWN:0002",
  "gene_name": "NADH dehydrogenase [ubiquinone] iron-sulfur protein 3, mitochondrial",
  "term_label": "Unknown biological process"
}